{
  "gene_name": "Serine palmitoyltransferase small subunit B",
  "gene": "UniProtKB:Q8NFR3",
  "gene_symbol": "SPTSSB",
  "term_id": "GO:0004758",
  "term_label": "serine C-palmitoyltransferase activity"
}